{
  "gene_symbol": "RPL18",
  "gene": "UniProtKB:Q07020",
  "gene_name": "Large ribosomal subunit protein eL18",
  "term_id": "GO:0003723",
  "term_label": "RNA binding"
}